{
  "gene_name": "Putative DENN domain-containing protein 10 B",
  "term_id": "GO:0031267",
  "gene_symbol": "DENND10P1",
  "term_label": "small GTPase binding",
  "gene": "UniProtKB:Q6NSW5"
}